{
  "gene": "UniProtKB:Q5T750",
  "gene_symbol": "KPLCE",
  "term_label": "Unknown cellular component",
  "term_id": "UNKNOWN:0003",
  "gene_name": "Protein KPLCE"
}